{
  "gene_symbol": "SLC12A8",
  "term_label": "potassium ion import across plasma membrane",
  "gene": "UniProtKB:A0AV02",
  "term_id": "GO:1990573",
  "gene_name": "Solute carrier family 12 member 8"
}